{
  "gene_name": "Zinc finger protein 775",
  "term_label": "RNA polymerase II cis-regulatory region sequence-specific DNA binding",
  "term_id": "GO:0000978",
  "gene": "UniProtKB:Q96BV0",
  "gene_symbol": "ZNF775"
}